{
  "term_id": "GO:0002365",
  "gene": "UniProtKB:Q4G0T1",
  "gene_symbol": "SCART1",
  "gene_name": "Scavenger receptor cysteine-rich domain-containing protein SCART1",
  "term_label": "gamma-delta T cell lineage commitment"
}